type I pilus [GO:0140621] (cellular component) References: PMID:28496159, PMID:29345620 Also known as: type 1 pilus, type I fimbriae, type I pili Definition: A short filamentous structure on the surface of a bacterial cell distinguished from other pili by their D-mannose-sensitive agglutinatination of erythrocytes. In E. coli, type I pili consist of a short tip fibrillum made up of the adhesin protein (FimH) and two minor subunits (FimG and FimF) that is joined to the pilus rod, a homopolymer of ~1000 FimA subunits. Relationships: is a type of pilus [GO:0009289]